{
  "term_id": "GO:0051896",
  "term_label": "regulation of phosphatidylinositol 3-kinase/protein kinase B signal transduction",
  "gene_name": "Divergent protein kinase domain 2A",
  "gene_symbol": "DIPK2A",
  "gene": "UniProtKB:Q8NDZ4"
}